{
  "gene_symbol": "CTAGE8",
  "term_label": "vesicle cargo loading",
  "gene": "UniProtKB:P0CG41",
  "gene_name": "cTAGE family member 8",
  "term_id": "GO:0035459"
}